{
  "gene_symbol": "OMD",
  "gene": "UniProtKB:Q99983",
  "term_id": "UNKNOWN:0002",
  "gene_name": "Osteomodulin",
  "term_label": "Unknown biological process"
}